{
  "gene": "UniProtKB:O76087",
  "term_id": "UNKNOWN:0002",
  "gene_symbol": "GAGE7",
  "term_label": "Unknown biological process",
  "gene_name": "G antigen 7"
}